{
  "term_id": "GO:0000978",
  "term_label": "RNA polymerase II cis-regulatory region sequence-specific DNA binding",
  "gene": "UniProtKB:Q86VE0",
  "gene_name": "Myb-related transcription factor, partner of profilin",
  "gene_symbol": "MYPOP"
}